{
  "term_id": "GO:0035267",
  "term_label": "NuA4 histone acetyltransferase complex",
  "gene_name": "YEATS domain-containing protein 2",
  "gene_symbol": "YEATS2",
  "gene": "UniProtKB:Q9ULM3"
}